{
  "gene_name": "TATA box-binding protein-like 1",
  "gene": "UniProtKB:P62380",
  "gene_symbol": "TBPL1",
  "term_id": "GO:0006352",
  "term_label": "DNA-templated transcription initiation"
}